{
  "term_label": "intracellular protein localization",
  "gene_symbol": "SEPTIN3",
  "gene": "UniProtKB:Q9UH03",
  "gene_name": "Neuronal-specific septin-3",
  "term_id": "GO:0008104"
}